{
  "gene": "UniProtKB:Q8WXD9",
  "gene_symbol": "CASKIN1",
  "term_label": "regulation of postsynaptic density assembly",
  "term_id": "GO:0099151",
  "gene_name": "Caskin-1"
}